{
  "term_label": "complement receptor activity",
  "gene_symbol": "GPR32",
  "gene": "UniProtKB:O75388",
  "term_id": "GO:0004875",
  "gene_name": "Probable G-protein coupled receptor 32"
}